{
  "term_label": "ATPase-coupled transmembrane transporter activity",
  "gene_symbol": "ABCA1",
  "term_id": "GO:0042626",
  "gene_name": "Phospholipid-transporting ATPase ABCA1",
  "gene": "UniProtKB:O95477"
}